{
  "gene_name": "Putative WAS protein family homolog 4",
  "term_id": "GO:0042147",
  "gene_symbol": "WASH4P",
  "gene": "UniProtKB:A8MWX3",
  "term_label": "retrograde transport, endosome to Golgi"
}